{
  "gene": "UniProtKB:P50583",
  "gene_symbol": "NUDT2",
  "term_id": "GO:0006167",
  "gene_name": "Bis(5'-nucleosyl)-tetraphosphatase [asymmetrical]",
  "term_label": "AMP biosynthetic process"
}